{
  "term_label": "fatty acid ligase activity",
  "gene_symbol": "ACSM4",
  "gene_name": "Acyl-coenzyme A synthetase ACSM4, mitochondrial",
  "term_id": "GO:0015645",
  "gene": "UniProtKB:P0C7M7"
}